early distal convoluted tubule development [GO:0072067] (biological process) Sources: GOC:mtg_kidney_jan10 Relationships: is a type of nephron epithelium development [GO:0072009]; is part of GO:0072025 Subtypes: metanephric early distal convoluted tubule development [GO:0072222] Definition: The process whose specific outcome is the progression of the early distal convoluted tubule over time, from its formation to the mature structure. The early distal convoluted tubule contains DCT cells and is vasopressin-insensitive.